{
  "gene": "UniProtKB:P47897",
  "term_id": "GO:0017101",
  "gene_name": "Glutamine--tRNA ligase",
  "term_label": "aminoacyl-tRNA synthetase multienzyme complex",
  "gene_symbol": "QARS1"
}